{
  "term_id": "GO:0051233",
  "term_label": "spindle midzone",
  "gene_symbol": "CENPV",
  "gene": "UniProtKB:Q7Z7K6",
  "gene_name": "Centromere protein V"
}